{
  "gene_symbol": "PDXDC2P",
  "gene_name": "Putative pyridoxal-dependent decarboxylase domain-containing protein 2",
  "term_label": "Unknown cellular component",
  "term_id": "UNKNOWN:0003",
  "gene": "UniProtKB:Q6P474"
}